DNA topoisomerase type II (double strand cut, ATP-hydrolyzing) regulator activity [GO:0072586] (molecular function) Definition: Binds to and modulates the activity of ATP-hydrolyzing DNA topoisomerase. DNA topoisomerase (ATP-hydrolyzing) regulator activity catalyzes a DNA topological transformation by transiently cleaving a pair of complementary DNA strands to form a gate through which a second double-stranded DNA segment is passed, after which the severed strands in the first DNA segment are rejoined; product release is coupled to ATP binding and hydrolysis; changes the linking number in multiples of 2. Sources: GOC:mah Subtypes: DNA topoisomerase type II (double strand cut, ATP-hydrolyzing) inhibitor activity [GO:0008657], DNA topoisomerase type II (double strand cut, ATP-hydrolyzing) activator activity [GO:0072587] Relationships: is_a enzyme regulator activity [GO:0030234]; is a type of ATPase regulator activity [GO:0060590]; regulates GO:0003918